{
  "term_label": "protein serine/threonine kinase activity",
  "gene_symbol": "STK16",
  "term_id": "GO:0004674",
  "gene": "UniProtKB:O75716",
  "gene_name": "Serine_threonine-protein kinase 16"
}